{
  "term_id": "GO:0005737",
  "gene": "UniProtKB:Q9UQL6",
  "term_label": "cytoplasm",
  "gene_name": "Histone deacetylase 5",
  "gene_symbol": "HDAC5"
}